{
  "gene_name": "Serpin I2",
  "term_label": "serine-type endopeptidase inhibitor activity",
  "gene": "UniProtKB:O75830",
  "gene_symbol": "SERPINI2",
  "term_id": "GO:0004867"
}